acylglycerol metabolic process [GO:0006639] (biological process) Sources: ISBN:0198506732 Definition: The chemical reactions and pathways involving acylglycerol, any mono-, di- or triester of glycerol with (one or more) fatty acids. Relationships: is a type of neutral lipid metabolic process [GO:0006638]; is a type of glycerolipid metabolic process [GO:0046486] Subtypes: triglyceride metabolic process [GO:0006641], acylglycerol acyl-chain remodeling [GO:0036155], diacylglycerol metabolic process [GO:0046339], monoacylglycerol metabolic process [GO:0046462], acylglycerol biosynthetic process [GO:0046463], acylglycerol catabolic process [GO:0046464] Also known as: acylglycerol metabolism, glyceride metabolic process, glyceride metabolism